{
  "term_label": "cyclin-dependent protein kinase holoenzyme complex",
  "term_id": "GO:0000307",
  "gene_symbol": "CDK17",
  "gene_name": "Cyclin-dependent kinase 17",
  "gene": "UniProtKB:Q00537"
}